{
  "gene_name": "Pleckstrin homology domain-containing family S member 1",
  "gene": "UniProtKB:Q5SXH7",
  "term_id": "UNKNOWN:0001",
  "term_label": "Unknown molecular function",
  "gene_symbol": "PLEKHS1"
}